activation of meiosis involved in egg activation [GO:0060466] (biological process) Sources: GOC:dph Relationships: is a type of activation of meiosis [GO:0090427]; is part of egg activation [GO:0007343] Also known as: resumption of meiosis involved in egg activation, reactivation of meiosis after fertilization Definition: Any process that starts the inactive process of meiosis in an egg after the egg has been fertilized or physiologically activated. Eggs generally arrest in meiosis and complete the process after activation.